{
  "term_id": "GO:0006955",
  "gene": "UniProtKB:Q7L513",
  "term_label": "immune response",
  "gene_symbol": "FCRLA",
  "gene_name": "Fc receptor-like A"
}